{
  "gene_name": "RNA-binding protein with multiple splicing 2",
  "term_id": "GO:0003729",
  "gene": "UniProtKB:Q6ZRY4",
  "term_label": "mRNA binding",
  "gene_symbol": "RBPMS2"
}